{
  "term_label": "Unknown biological process",
  "term_id": "UNKNOWN:0002",
  "gene_name": "Putative uncharacterized protein MGC163334",
  "gene_symbol": "Q5W150",
  "gene": "UniProtKB:Q5W150"
}